AV node cell to bundle of His cell communication [GO:0086067] (biological process) Sources: GOC:BHF, GOC:mtg_cardiac_conduct_nov11 Relationships: is a type of GO:0086065 Also known as: atrioventricular node cell to bundle of His cell communication Definition: The process that mediates interactions between an AV node cell and its surroundings that contributes to the process of the AV node cell communicating with a bundle of His cell in cardiac conduction. Encompasses interactions such as signaling or attachment between one cell and another cell, between a cell and an extracellular matrix, or between a cell and any other aspect of its environment. Subtypes: AV node cell to bundle of His cell signaling [GO:0086027], GO:0086053